{
  "gene_symbol": "FAM217B",
  "term_id": "UNKNOWN:0001",
  "term_label": "Unknown molecular function",
  "gene_name": "Protein FAM217B",
  "gene": "UniProtKB:Q9NTX9"
}